{
  "gene": "UniProtKB:Q9Y3C5",
  "gene_name": "RING finger protein 11",
  "term_id": "GO:0006511",
  "term_label": "ubiquitin-dependent protein catabolic process",
  "gene_symbol": "RNF11"
}